{
  "gene_name": "Putative monooxygenase p33MONOX",
  "term_id": "UNKNOWN:0001",
  "gene": "UniProtKB:Q96A73",
  "gene_symbol": "KIAA1191",
  "term_label": "Unknown molecular function"
}